{
  "gene_symbol": "FAM167A",
  "term_id": "UNKNOWN:0002",
  "gene": "UniProtKB:Q96KS9",
  "gene_name": "Protein FAM167A",
  "term_label": "Unknown biological process"
}